inflammatory response to antigenic stimulus [GO:0002437] (biological process) Regulation: RO_0002211 by regulation of inflammatory response to antigenic stimulus [GO:0002861]; negatively regulated by negative regulation of inflammatory response to antigenic stimulus [GO:0002862]; positively regulated by GO:0002863 Relationships: is a type of inflammatory response [GO:0006954]; is a type of immune response [GO:0006955] Subtypes: acute inflammatory response to antigenic stimulus [GO:0002438], chronic inflammatory response to antigenic stimulus [GO:0002439], histamine secretion mediated by immunoglobulin [GO:0097280] Sources: GOC:add, ISBN:0781735149 Definition: An inflammatory response to an antigenic stimulus, which can be include any number of T cell or B cell epitopes.